{
  "gene_symbol": "H2BC13",
  "gene": "UniProtKB:Q99880",
  "term_label": "nucleus",
  "term_id": "GO:0005634",
  "gene_name": "Histone H2B type 1-L"
}